{
  "gene_name": "MANSC domain-containing protein 1",
  "gene_symbol": "MANSC1",
  "gene": "UniProtKB:Q9H8J5",
  "term_id": "GO:0005794",
  "term_label": "Golgi apparatus"
}